inner kinetochore [GO:0000939] (cellular component) Also known as: condensed chromosome inner kinetochore, condensed nuclear chromosome inner kinetochore, inner kinetochore of condensed chromosome, inner kinetochore of condensed nuclear chromosome, inner kinetochore plate, inner centromere core complex Definition: The region of a kinetochore closest to centromeric DNA which contains many CENP proteins organized in various subcomplexes including CENP-C, CENP-LN, CENP-HIKM, CENP-OPQUR and CENP-TWSX, but excluding the CENP-A containing heterochromatin. Relationships: is a type of protein-containing complex [GO:0032991]; is part of GO:0000776 References: PMID:10619130, PMID:11483983, PMID:32516549 Sources: GOC:clt